sterol 12-alpha-hydroxylase activity [GO:0008397] (molecular function) Definition: Catalysis of the reaction: a steroid + reduced [NADPH--hemoprotein reductase] + O2 = a 12-alpha-hydroxysteroid + oxidized [NADPH--hemoprotein reductase]- H2O +H+. Relationships: is a type of steroid hydroxylase activity [GO:0008395]; is a type of oxidoreductase activity, acting on paired donors, with incorporation or reduction of molecular oxygen, reduced flavin or flavoprotein as one donor, and incorporation of one atom of oxygen [GO:0016712] Also known as: cytochrome P450 CYP8B1 Sources: EC:1.14.14.139